{
  "gene": "UniProtKB:Q92581",
  "term_label": "sodium ion import across plasma membrane",
  "gene_name": "Sodium_hydrogen exchanger 6",
  "term_id": "GO:0098719",
  "gene_symbol": "SLC9A6"
}